3'-demethylstaurosporine O-methyltransferase activity [GO:0030793] (molecular function) Definition: Catalysis of the reaction: 3'-demethylstaurosporine + S-adenosyl-L-methionine = S-adenosyl-L-homocysteine + H+ + staurosporine. Also known as: 3'-demethoxy-3'-hydroxystaurosporine O-methyltransferase activity, S-adenosyl-L-methionine:3'-demethylstaurosporine O-methyltransferase activity, staurosporine synthase activity Sources: EC:2.1.1.139, RHEA:11696 Relationships: is a type of GO:0008757